cartilage morphogenesis [GO:0060536] (biological process) Definition: The process in which the anatomical structures of cartilage are generated and organized. Subtypes: growth plate cartilage morphogenesis [GO:0003422], GO:0060533, trachea cartilage morphogenesis [GO:0060535] Relationships: is a type of animal organ morphogenesis [GO:0009887]; is a type of tissue morphogenesis [GO:0048729]; is part of cartilage development [GO:0051216] Sources: GOC:dph